small conductance calcium-activated potassium channel inhibitor activity [GO:0140629] (molecular function) Definition: Binds to and stops, prevents, or reduces the activity of a small conductance calcium-activated potassium channel. References: PMID:20562108 Relationships: is a type of potassium channel inhibitor activity [GO:0019870]; negatively regulates small conductance calcium-activated potassium channel activity [GO:0016286]